{
  "term_id": "GO:0005243",
  "gene_name": "Gap junction alpha-9 protein",
  "term_label": "gap junction channel activity",
  "gene": "UniProtKB:P57773",
  "gene_symbol": "GJA9"
}